wobble position uridine ribose methylation [GO:0002132] (biological process) Relationships: is a type of GO:0002130 Definition: The process in which the ribose of uridine at position 34 in the anticodon of a tRNA is post-transcriptionally methylated at the 2'-O position. Sources: GOC:hjd, ISBN:155581073X